{
  "gene": "UniProtKB:P47804",
  "gene_symbol": "RGR",
  "term_label": "plasma membrane",
  "gene_name": "RPE-retinal G protein-coupled receptor",
  "term_id": "GO:0005886"
}